{
  "term_id": "UNKNOWN:0001",
  "term_label": "Unknown molecular function",
  "gene_name": "BRO1 domain-containing protein BROX",
  "gene_symbol": "BROX",
  "gene": "UniProtKB:Q5VW32"
}